cellular response to aldehyde [GO:0110096] (biological process) Definition: Any process that results in a change in state or activity of a cell (in terms of movement, secretion, enzyme production, gene expression, etc.) as a result of an aldehyde stimulus. References: PMID:25656103 Sources: GOC:vw Relationships: is a type of cellular response to oxygen-containing compound [GO:1901701] Subtypes: cellular response to glyoxal [GO:0036471], cellular response to methylglyoxal [GO:0097238], cellular response to aldosterone [GO:1904045], cellular response to formaldehyde [GO:1904405], cellular response to acetaldehyde [GO:1905641]